{
  "gene_name": "Coiled-coil domain-containing protein 71L",
  "gene_symbol": "CCDC71L",
  "gene": "UniProtKB:Q8N9Z2",
  "term_id": "UNKNOWN:0001",
  "term_label": "Unknown molecular function"
}